{
  "gene_symbol": "PSME1",
  "term_id": "GO:2000045",
  "gene": "UniProtKB:Q06323",
  "gene_name": "Proteasome activator complex subunit 1",
  "term_label": "regulation of G1/S transition of mitotic cell cycle"
}